gamma-tubulin ring complex [GO:0000931] (cellular component) Definition: A complex of gamma tubulin and associated proteins thought to be formed by multimerization of gamma-tubulin small complexes. An example of this structure is found in Schizosaccharomyces pombe. References: PMID:12134075, PMID:17021256 Sources: GOC:mtg_sensu Relationships: is a type of gamma-tubulin complex [GO:0000930]; has part gamma-tubulin small complex [GO:0008275] Also known as: gamma-TuRC, gamma-tubulin large complex, centrosomal, gamma-tubulin large complex, eMTOC, gamma-tubulin large complex, equatorial microtubule organizing center, gamma-tubulin large complex, equatorial microtubule organizing centre, gamma-tubulin large complex, iMTOC, gamma-tubulin large complex, interphase microtubule organizing center, gamma-tubulin large complex, interphase microtubule organizing centre, gamma-tubulin large complex, mitotic spindle pole body, gamma-tubulin large complex, spindle pole body, gamma-tubulin ring complex, centrosomal, gamma-tubulin large complex